sensory perception of chemical stimulus [GO:0007606] (biological process) Also known as: chemosensory perception Relationships: is a type of sensory perception [GO:0007600] Sources: GOC:ai Definition: The series of events required for an organism to receive a sensory chemical stimulus, convert it to a molecular signal, and recognize and characterize the signal. This is a neurological process. Subtypes: sensory perception of smell [GO:0007608], sensory perception of taste [GO:0050909], magnetoreception by sensory perception of chemical stimulus [GO:0050977]